{
  "gene_name": "Putative uncharacterized protein SLC66A1L",
  "term_label": "Unknown biological process",
  "gene": "UniProtKB:A1A4F0",
  "gene_symbol": "SLC66A1LP",
  "term_id": "UNKNOWN:0002"
}